gallbladder development [GO:0061010] (biological process) Sources: GOC:dph Definition: The progression of the gallbladder over time, from its initial formation to the mature structure. The gallbladder is a cavitated organ that stores bile. Relationships: is a type of animal organ development [GO:0048513]; is part of hepaticobiliary system development [GO:0061008]